{
  "gene": "UniProtKB:Q96LW4",
  "gene_symbol": "PRIMPOL",
  "term_id": "GO:0031297",
  "term_label": "replication fork processing",
  "gene_name": "DNA-directed primase_polymerase protein"
}